{
  "term_id": "GO:0005886",
  "gene_symbol": "DTNBP1",
  "term_label": "plasma membrane",
  "gene_name": "Dysbindin",
  "gene": "UniProtKB:Q96EV8"
}